cerebellar climbing fiber to Purkinje cell synapse [GO:0150053] (cellular component) Definition: A synapse of a climbing fiber onto the dendrites of a Purkinje cell in cerebellum. The climbing fiber originates from the inferior olivary nucleus of the medulla oblongata. References: PMID:19597563, PMID:23811844, PMID:5044254 Sources: GOC:aruk, GOC:bc Also known as: cerebellar climbing fibre to Purkinje cell synapse Relationships: is a type of asymmetric, glutamatergic, excitatory synapse [GO:0098985]